{
  "term_label": "RNA polymerase II cis-regulatory region sequence-specific DNA binding",
  "gene_name": "Chorion-specific transcription factor GCMb",
  "term_id": "GO:0000978",
  "gene_symbol": "GCM2",
  "gene": "UniProtKB:O75603"
}